{
  "gene_symbol": "MED15",
  "gene": "UniProtKB:Q96RN5",
  "term_label": "Unknown biological process",
  "gene_name": "Mediator of RNA polymerase II transcription subunit 15",
  "term_id": "UNKNOWN:0002"
}